{
  "term_label": "cytoplasm",
  "gene_symbol": "MYL12A",
  "gene_name": "Myosin regulatory light chain 12A",
  "term_id": "GO:0005737",
  "gene": "UniProtKB:P19105"
}